{
  "gene_name": "WD repeat, SAM and U-box domain-containing protein 1",
  "term_id": "UNKNOWN:0001",
  "gene_symbol": "WDSUB1",
  "term_label": "Unknown molecular function",
  "gene": "UniProtKB:Q8N9V3"
}